{
  "gene_symbol": "CHRNB3",
  "term_id": "GO:0005892",
  "gene": "UniProtKB:Q05901",
  "term_label": "acetylcholine-gated channel complex",
  "gene_name": "Neuronal acetylcholine receptor subunit beta-3"
}